{
  "gene": "UniProtKB:Q8N3R9",
  "term_id": "GO:0002011",
  "gene_symbol": "PALS1",
  "gene_name": "Protein PALS1",
  "term_label": "morphogenesis of an epithelial sheet"
}